{
  "term_label": "rRNA processing",
  "term_id": "GO:0006364",
  "gene_symbol": "WDR18",
  "gene": "UniProtKB:Q9BV38",
  "gene_name": "WD repeat-containing protein 18"
}